{
  "gene": "UniProtKB:P84095",
  "gene_symbol": "RHOG",
  "term_label": "regulation of actin cytoskeleton organization",
  "term_id": "GO:0032956",
  "gene_name": "Rho-related GTP-binding protein RhoG"
}